{
  "gene": "UniProtKB:P31275",
  "term_id": "UNKNOWN:0003",
  "gene_symbol": "HOXC12",
  "term_label": "Unknown cellular component",
  "gene_name": "Homeobox protein Hox-C12"
}